{
  "gene": "UniProtKB:P08069",
  "gene_name": "Insulin-like growth factor 1 receptor",
  "term_id": "GO:0008286",
  "gene_symbol": "IGF1R",
  "term_label": "insulin receptor signaling pathway"
}